{
  "gene_symbol": "DPH2",
  "gene": "UniProtKB:Q9BQC3",
  "gene_name": "2-(3-amino-3-carboxypropyl)histidine synthase subunit 2",
  "term_id": "UNKNOWN:0001",
  "term_label": "Unknown molecular function"
}